{
  "gene": "UniProtKB:P19784",
  "term_id": "GO:0005634",
  "gene_name": "Casein kinase II subunit alpha'",
  "gene_symbol": "CSNK2A2",
  "term_label": "nucleus"
}